major mitochondrial derivative [GO:0016008] (cellular component) Relationships: is a type of mitochondrial derivative [GO:0016007] References: PMID:17123504, PMID:24211517, PMID:30802236 Sources: GOC:mah Definition: The larger of the two mitochondrial derivatives that arise by the unfolding of the Nebenkern during flagellum elongation; the major mitochondrial derivative is ovoid and darker than the minor derivative.